intrachromosomal DNA recombination [GO:1990067] (biological process) Also known as: intrastrand DNA recombination Relationships: is a type of GO:0006310 References: PMID:7748165 Definition: The process of DNA recombination occurring within a single chromosome.